{
  "term_label": "1-phosphatidylinositol-3-kinase regulator activity",
  "gene": "UniProtKB:Q8WYR1",
  "gene_symbol": "PIK3R5",
  "term_id": "GO:0046935",
  "gene_name": "Phosphoinositide 3-kinase regulatory subunit 5"
}